{
  "term_label": "Unknown molecular function",
  "gene": "UniProtKB:Q86XP3",
  "gene_symbol": "DDX42",
  "gene_name": "ATP-dependent RNA helicase DDX42",
  "term_id": "UNKNOWN:0001"
}